regulation of DNA replication initiation involved in plasmid copy number maintenance [GO:0060909] (biological process) Subtypes: negative regulation of DNA replication initiation involved in plasmid copy number maintenance [GO:0060910] Relationships: is a type of GO:0030174; is part of plasmid copy number maintenance [GO:0060908] Sources: GOC:dph, GOC:tb Definition: Any process that modulates the frequency, rate or extent of initiation of plasmid DNA replication that contributes to copy number maintenance.